regulation of cellular response to osmotic stress [GO:0106049] (biological process) Definition: Any process that modulates the frequency, rate or extent of the cellular response to osmotic stress. Relationships: is_a GO:0047484; is a type of GO:0080135; regulates GO:0071470 References: PMID:10398679 Subtypes: regulation of cellular hyperosmotic salinity response [GO:1900069], regulation of intrinsic apoptotic signaling pathway in response to osmotic stress [GO:1902218]